{
  "term_label": "Unknown biological process",
  "gene": "UniProtKB:P04090",
  "term_id": "UNKNOWN:0002",
  "gene_name": "Prorelaxin H2",
  "gene_symbol": "RLN2"
}